{
  "gene_symbol": "NR2F6",
  "term_id": "GO:0007399",
  "gene": "UniProtKB:P10588",
  "term_label": "nervous system development",
  "gene_name": "Nuclear receptor subfamily 2 group F member 6"
}